{
  "term_id": "GO:0016485",
  "term_label": "protein processing",
  "gene_name": "Suppressor of tumorigenicity 14 protein",
  "gene": "UniProtKB:Q9Y5Y6",
  "gene_symbol": "ST14"
}